telomere formation via telomerase [GO:0032203] (BP) Definition: A cellular process that results in the formation of a telomere at a non-telomeric double-stranded DNA end that involves the activity of a telomerase enzyme. Relationships: is a type of telomere assembly [GO:0032202]; has part telomerase activity [GO:0003720]; has part GO:1905324 References: PMID:11902675, PMID:8622671 Sources: GOC:cjm, GOC:ns